{
  "term_id": "GO:0046856",
  "term_label": "phosphatidylinositol dephosphorylation",
  "gene_symbol": "PIP4P1",
  "gene_name": "Type 1 phosphatidylinositol 4,5-bisphosphate 4-phosphatase",
  "gene": "UniProtKB:Q86T03"
}